{
  "gene_name": "B-cell receptor CD22",
  "gene": "UniProtKB:P20273",
  "term_label": "early endosome",
  "gene_symbol": "CD22",
  "term_id": "GO:0005769"
}